{
  "term_id": "GO:0006357",
  "gene": "UniProtKB:Q8TF68",
  "gene_symbol": "ZNF384",
  "gene_name": "Zinc finger protein 384",
  "term_label": "regulation of transcription by RNA polymerase II"
}